{
  "gene_name": "YTH domain-containing family protein 1",
  "gene_symbol": "YTHDF1",
  "gene": "UniProtKB:Q9BYJ9",
  "term_id": "GO:0061157",
  "term_label": "mRNA destabilization"
}